{
  "term_id": "GO:0047453",
  "gene_symbol": "NAXD",
  "term_label": "ATP-dependent NAD(P)H-hydrate dehydratase activity",
  "gene": "UniProtKB:Q8IW45",
  "gene_name": "ATP-dependent (S)-NAD(P)H-hydrate dehydratase"
}